{
  "gene_symbol": "TEX22",
  "term_id": "UNKNOWN:0003",
  "gene_name": "Testis-expressed protein 22",
  "gene": "UniProtKB:C9J3V5",
  "term_label": "Unknown cellular component"
}